protein localization to mitotic spindle [GO:1902480] (biological process) Relationships: is a type of GO:0072698 Definition: A process in which a protein is transported to, or maintained in, a location within a mitotic spindle. Also known as: protein localisation in mitotic spindle, protein localisation to mitotic spindle, protein localization in mitotic spindle Subtypes: protein localization to mitotic spindle midzone [GO:1902967] References: PMID:23885124 Sources: GOC:TermGenie